proteoglycan binding [GO:0043394] (molecular function) Sources: ISBN:0198506732 Relationships: is a type of GO:0005515; is a type of carbohydrate derivative binding [GO:0097367] Subtypes: chondroitin sulfate proteoglycan binding [GO:0035373], heparan sulfate proteoglycan binding [GO:0043395], syndecan binding [GO:0045545] Definition: Binding to a proteoglycan, any glycoprotein in which the carbohydrate units are glycosaminoglycans.